{
  "term_label": "tRNA (guanine(46)-N7)-methyltransferase activity",
  "gene_symbol": "METTL1",
  "gene": "UniProtKB:Q9UBP6",
  "term_id": "GO:0008176",
  "gene_name": "tRNA (guanine-N(7)-)-methyltransferase"
}